{
  "gene": "UniProtKB:O15229",
  "gene_name": "Kynurenine 3-monooxygenase",
  "gene_symbol": "KMO",
  "term_id": "GO:0004502",
  "term_label": "kynurenine 3-monooxygenase activity"
}